{
  "term_label": "Unknown molecular function",
  "gene_name": "Uncharacterized protein",
  "term_id": "UNKNOWN:0001",
  "gene": "UniProtKB:A0A8V8TPC4",
  "gene_symbol": "A0A8V8TPC4"
}